{
  "term_id": "UNKNOWN:0002",
  "gene_symbol": "FGD6",
  "gene": "UniProtKB:Q6ZV73",
  "term_label": "Unknown biological process",
  "gene_name": "FYVE, RhoGEF and PH domain-containing protein 6"
}